positive regulation of interleukin-33 production [GO:0150129] (biological process) Definition: Any process that activates or increases the frequency, rate or extent of interleukin-33 production. Relationships: is a type of GO:0001819; is a type of regulation of interleukin-33 production [GO:0150127]; positively regulates GO:0072639 Also known as: positive regulation of interleukin-33 biosynthetic process, positive regulation of interleukin-33 secretion Sources: GOC:aruk